neuron fate specification [GO:0048665] (biological process) Definition: The process in which a cell becomes capable of differentiating autonomously into a neuron in an environment that is neutral with respect to the developmental pathway. Upon specification, the cell fate can be reversed. Subtypes: GO:0021518, spinal cord association neuron specification [GO:0021519], spinal cord motor neuron cell fate specification [GO:0021520], ventral spinal cord interneuron specification [GO:0021521], auditory receptor cell fate specification [GO:0042667], photoreceptor cell fate specification [GO:0043704] Relationships: is a type of cell fate specification [GO:0001708]; is part of neuron fate commitment [GO:0048663] Sources: GOC:dph